{
  "gene_symbol": "ANKRD1",
  "term_id": "GO:0061629",
  "gene_name": "Ankyrin repeat domain-containing protein 1",
  "gene": "UniProtKB:Q15327",
  "term_label": "RNA polymerase II-specific DNA-binding transcription factor binding"
}